{
  "gene": "UniProtKB:Q52LR7",
  "gene_name": "Enhancer of polycomb homolog 2",
  "gene_symbol": "EPC2",
  "term_id": "GO:0035267",
  "term_label": "NuA4 histone acetyltransferase complex"
}